{
  "gene": "UniProtKB:Q9NUQ7",
  "term_label": "endoplasmic reticulum",
  "gene_symbol": "UFSP2",
  "gene_name": "Ufm1-specific protease 2",
  "term_id": "GO:0005783"
}